{
  "gene": "UniProtKB:Q8NH73",
  "term_label": "olfactory receptor activity",
  "gene_name": "Olfactory receptor 4S2",
  "gene_symbol": "OR4S2",
  "term_id": "GO:0004984"
}